{
  "gene_name": "Uncharacterized protein C19orf85",
  "gene_symbol": "C19orf85",
  "term_label": "Unknown cellular component",
  "term_id": "UNKNOWN:0003",
  "gene": "UniProtKB:A0A1B0GUS0"
}